{
  "term_label": "G protein-coupled GABA receptor activity",
  "gene_name": "Gamma-aminobutyric acid type B receptor subunit 1",
  "term_id": "GO:0004965",
  "gene": "UniProtKB:Q9UBS5",
  "gene_symbol": "GABBR1"
}